inferior salivary nucleus development [GO:0021752] (biological process) Sources: GOC:cls, GOC:curators, GOC:dgh, GOC:dph, GOC:jid Definition: The process whose specific outcome is the progression of the inferior salivary nucleus over time, from its formation to the mature structure. Relationships: is a type of salivary nucleus development [GO:0021751]